Wnt protein secretion [GO:0061355] (biological process) Definition: The controlled release of a Wnt protein from a cell. References: PMID:19223472 Sources: GOC:bf Relationships: is a type of GO:0009306; is a type of signal release [GO:0023061] Regulation: regulated by regulation of Wnt protein secretion [GO:0061356]; positively regulated by GO:0061357; negatively regulated by negative regulation of Wnt protein secretion [GO:0061358]